{
  "gene_name": "Olfactory receptor 1J4",
  "term_label": "olfactory receptor activity",
  "gene_symbol": "OR1J4",
  "gene": "UniProtKB:Q8NGS1",
  "term_id": "GO:0004984"
}